{
  "term_label": "U2 snRNP",
  "gene_name": "Small nuclear ribonucleoprotein Sm D1",
  "gene_symbol": "SNRPD1",
  "term_id": "GO:0005686",
  "gene": "UniProtKB:P62314"
}